regulation of unidimensional cell growth [GO:0051510] (biological process) Subtypes: negative regulation of unidimensional cell growth [GO:0051511], positive regulation of unidimensional cell growth [GO:0051512], regulation of monopolar cell growth [GO:0051513], regulation of bipolar cell growth [GO:0051516], regulation of pollen tube growth [GO:0080092] Also known as: regulation of cell elongation Sources: GOC:ai Definition: Any process that modulates the frequency, rate or extent of unidimensional cell growth, the process in which a cell irreversibly increases in size in one [spatial] dimension or along one axis. Relationships: is a type of regulation of cell growth [GO:0001558]; is a type of regulation of cell morphogenesis [GO:0022604]; is a type of GO:0048638; RO_0002211 unidimensional cell growth [GO:0009826]